{
  "gene_name": "Transmembrane protease serine 2",
  "term_label": "plasma membrane",
  "gene_symbol": "TMPRSS2",
  "term_id": "GO:0005886",
  "gene": "UniProtKB:O15393"
}